{
  "term_label": "poly-N-acetyllactosamine biosynthetic process",
  "gene_symbol": "B3GNT9",
  "gene_name": "UDP-GlcNAc:betaGal beta-1,3-N-acetylglucosaminyltransferase 9",
  "term_id": "GO:0030311",
  "gene": "UniProtKB:Q6UX72"
}